{
  "term_id": "UNKNOWN:0001",
  "gene_symbol": "ZER1",
  "gene_name": "Protein zer-1 homolog",
  "term_label": "Unknown molecular function",
  "gene": "UniProtKB:Q7Z7L7"
}